negative regulation of heme biosynthetic process [GO:0070454] (biological process) Definition: Any process that decreases the frequency, rate or extent of the chemical reactions and pathways resulting in the formation of heme. Sources: GOC:mah Also known as: down regulation of heme biosynthetic process, down-regulation of heme biosynthetic process, downregulation of heme biosynthetic process, negative regulation of haem biosynthetic process, negative regulation of heme anabolism, negative regulation of heme biosynthesis, negative regulation of heme formation, negative regulation of heme synthesis, inhibition of heme biosynthetic process Relationships: is a type of regulation of heme biosynthetic process [GO:0070453]; is a type of negative regulation of tetrapyrrole biosynthetic process [GO:1901464]; negatively regulates heme biosynthetic process [GO:0006783]